{
  "term_label": "cellular response to heat",
  "term_id": "GO:0034605",
  "gene_name": "DnaJ homolog subfamily A member 2",
  "gene_symbol": "DNAJA2",
  "gene": "UniProtKB:O60884"
}